{
  "term_label": "Unknown cellular component",
  "gene_name": "Heparan sulfate glucosamine 3-O-sulfotransferase 3B1",
  "term_id": "UNKNOWN:0003",
  "gene_symbol": "HS3ST3B1",
  "gene": "UniProtKB:Q9Y662"
}